negative regulation of flagellated sperm motility [GO:1901318] (biological process) Definition: Any process that stops, prevents or reduces the frequency, rate or extent of flagellated sperm motility. Sources: GOC:TermGenie, GOC:cilia, GOC:krc Also known as: down regulation of sperm motility, down regulation of sperm movement, down-regulation of sperm motility, down-regulation of sperm movement, downregulation of sperm motility, downregulation of sperm movement, inhibition of sperm movement, negative regulation of sperm motility, negative regulation of sperm movement, inhibition of sperm motility Relationships: is a type of negative regulation of cilium movement [GO:0003354]; is a type of GO:1901317; is_a negative regulation of cilium-dependent cell motility [GO:1902020]; is a type of negative regulation of reproductive process [GO:2000242]; negatively regulates flagellated sperm motility [GO:0030317]